{
  "gene_name": "C-type lectin domain family 4 member D",
  "gene": "UniProtKB:Q8WXI8",
  "term_label": "carbohydrate binding",
  "gene_symbol": "CLEC4D",
  "term_id": "GO:0030246"
}